{
  "gene_name": "Secretagogin",
  "gene": "UniProtKB:O76038",
  "term_id": "GO:0005829",
  "gene_symbol": "SCGN",
  "term_label": "cytosol"
}